{
  "term_label": "enzyme activator activity",
  "gene": "UniProtKB:Q9BTL3",
  "gene_symbol": "RAMAC",
  "term_id": "GO:0008047",
  "gene_name": "RNA guanine-N7 methyltransferase activating subunit"
}